{
  "gene_symbol": "WWC1",
  "gene_name": "Protein KIBRA",
  "term_id": "GO:0019900",
  "term_label": "kinase binding",
  "gene": "UniProtKB:Q8IX03"
}